{
  "term_id": "GO:0030425",
  "gene_name": "5-hydroxytryptamine receptor 1E",
  "gene": "UniProtKB:P28566",
  "term_label": "dendrite",
  "gene_symbol": "HTR1E"
}